{
  "gene_name": "Proto-oncogene Mas",
  "gene": "UniProtKB:P04201",
  "term_id": "GO:0007186",
  "term_label": "G protein-coupled receptor signaling pathway",
  "gene_symbol": "MAS1"
}